{
  "term_id": "GO:0008143",
  "gene_symbol": "KHDRBS2",
  "gene": "UniProtKB:Q5VWX1",
  "term_label": "poly(A) binding",
  "gene_name": "KH domain-containing, RNA-binding, signal transduction-associated protein 2"
}